{
  "gene_symbol": "NPIPB4",
  "gene_name": "Nuclear pore complex-interacting protein family member B4",
  "term_id": "UNKNOWN:0002",
  "term_label": "Unknown biological process",
  "gene": "UniProtKB:C9JG80"
}